{
  "gene_symbol": "ZNF772",
  "term_id": "GO:0000981",
  "gene_name": "Zinc finger protein 772",
  "term_label": "DNA-binding transcription factor activity, RNA polymerase II-specific",
  "gene": "UniProtKB:Q68DY9"
}